neuron recognition [GO:0008038] (biological process) Definition: The process in which a neuronal cell in a multicellular organism interprets its surroundings. Subtypes: axonal fasciculation [GO:0007413], axonal defasciculation [GO:0007414], synaptic target recognition [GO:0008039], axon choice point recognition [GO:0016198], dendrite self-avoidance [GO:0070593] Relationships: is a type of cell recognition [GO:0008037]; is part of neuron development [GO:0048666] Sources: GOC:go_curators Also known as: neuronal cell recognition